regulation of protein catabolic process in the vacuole [GO:1904350] (biological process) Relationships: is_a regulation of protein catabolic process [GO:0042176]; regulates protein catabolic process in the vacuole [GO:0007039] References: PMID:25635054 Sources: GOC:BHF, GOC:TermGenie, GOC:rl, GO_REF:0000058 Also known as: regulation of vacuolar protein breakdown, regulation of vacuolar protein catabolic process, regulation of vacuolar protein catabolism, regulation of vacuolar protein degradation Subtypes: negative regulation of protein catabolic process in the vacuole [GO:1904351], positive regulation of protein catabolic process in the vacuole [GO:1904352], regulation of lysosomal protein catabolic process [GO:1905165] Definition: Any process that modulates the frequency, rate or extent of protein catabolic process in the vacuole.